cellular response to serotonin [GO:1904015] (biological process) References: PMID:1505525 Sources: GOC:TermGenie, GO_REF:0000071 Definition: Any process that results in a change in state or activity of a cell (in terms of movement, secretion, enzyme production, gene expression, etc.) as a result of a serotonin stimulus. Relationships: is a type of cellular response to monoamine stimulus [GO:0071868]; is_a cellular response to oxygen-containing compound [GO:1901701]; is_a response to serotonin [GO:1904014]